{
  "term_id": "GO:0048179",
  "gene_symbol": "TGFBR1",
  "term_label": "activin receptor complex",
  "gene_name": "TGF-beta receptor type-1",
  "gene": "UniProtKB:P36897"
}